{
  "term_label": "Unknown biological process",
  "gene_symbol": "CTXND1",
  "gene_name": "Cortexin domain-containing 1 protein",
  "term_id": "UNKNOWN:0002",
  "gene": "UniProtKB:A0A1B0GTU2"
}